{
  "term_id": "GO:0005886",
  "gene": "UniProtKB:P09601",
  "gene_symbol": "HMOX1",
  "term_label": "plasma membrane",
  "gene_name": "Heme oxygenase 1"
}